{
  "gene": "UniProtKB:Q6ZMR3",
  "gene_name": "L-lactate dehydrogenase A-like 6A",
  "term_label": "pyruvate catabolic process",
  "term_id": "GO:0042867",
  "gene_symbol": "LDHAL6A"
}